{
  "gene_symbol": "EXOC3-AS1",
  "term_id": "UNKNOWN:0002",
  "gene": "UniProtKB:Q8N2X6",
  "term_label": "Unknown biological process",
  "gene_name": "Uncharacterized protein EXOC3-AS1"
}